positive regulation of eosinophil extravasation [GO:2000421] (biological process) Sources: GOC:BHF, GOC:mah Definition: Any process that activates or increases the frequency, rate or extent of eosinophil extravasation. Relationships: is a type of GO:0002693; is a type of positive regulation of eosinophil migration [GO:2000418]; is a type of regulation of eosinophil extravasation [GO:2000419]; positively regulates eosinophil extravasation [GO:0072682]